{
  "gene_name": "Peroxisomal testis-specific protein 1",
  "term_id": "UNKNOWN:0003",
  "gene_symbol": "PXT1",
  "gene": "UniProtKB:Q8NFP0",
  "term_label": "Unknown cellular component"
}